{
  "gene": "UniProtKB:P0DPK5",
  "term_label": "nucleus",
  "gene_name": "Histone H3.X",
  "term_id": "GO:0005634",
  "gene_symbol": "H3Y2"
}